{
  "gene_name": "Keratin-associated protein 19-2",
  "gene": "UniProtKB:Q3LHN2",
  "term_label": "Unknown molecular function",
  "gene_symbol": "KRTAP19-2",
  "term_id": "UNKNOWN:0001"
}